{
  "term_label": "transcription regulator complex",
  "gene_name": "Mitotic deacetylase-associated SANT domain protein",
  "gene_symbol": "MIDEAS",
  "gene": "UniProtKB:Q6PJG2",
  "term_id": "GO:0005667"
}